tRNA 5'-leader removal [GO:0001682] (biological process) Definition: Generation of the mature 5'-end of the tRNA, usually via an endonucleolytic cleavage by RNase P. Relationships: is a type of tRNA 5'-end processing [GO:0099116] References: PMID:11592395 Also known as: tRNA 5' leader removal